{
  "term_id": "GO:0003682",
  "gene_symbol": "CBX3",
  "gene_name": "Chromobox protein homolog 3",
  "gene": "UniProtKB:Q13185",
  "term_label": "chromatin binding"
}